regulation of smooth muscle contraction [GO:0006940] (biological process) Definition: Any process that modulates the frequency, rate or extent of smooth muscle contraction. Subtypes: GO:0003056, regulation of hindgut contraction [GO:0043134], negative regulation of smooth muscle contraction [GO:0045986], GO:0045987, GO:0070472, regulation of gastro-intestinal system smooth muscle contraction [GO:1904304], GO:1904318 Relationships: is a type of regulation of muscle contraction [GO:0006937]; regulates smooth muscle contraction [GO:0006939] Sources: GOC:go_curators